{
  "gene_name": "RAS protein activator like-3",
  "term_id": "GO:1902531",
  "gene_symbol": "RASAL3",
  "term_label": "regulation of intracellular signal transduction",
  "gene": "UniProtKB:Q86YV0"
}